tRNA queuosine(34) biosynthetic process from salvaged queuosine or its precursors [GO:0160254] (biological process) Definition: The chemical reactions and pathways resulting in the formation of tRNA queuosine(34) by salvaging available queuosine or precursors of queuosine (preQ0 or preQ1). References: PMID:28208705, PMID:39600051 Sources: MetaCyc:PWY-8106 Relationships: is a type of tRNA queuosine(34) biosynthetic process [GO:0008616]